{
  "gene_symbol": "SLITRK6",
  "term_label": "plasma membrane",
  "gene": "UniProtKB:Q9H5Y7",
  "gene_name": "SLIT and NTRK-like protein 6",
  "term_id": "GO:0005886"
}